{
  "term_label": "lysosomal membrane",
  "term_id": "GO:0005765",
  "gene_name": "Mucolipin-1",
  "gene_symbol": "MCOLN1",
  "gene": "UniProtKB:Q9GZU1"
}